alphaIIb-beta3 integrin-talin complex [GO:0070515] (cellular component) References: PMID:8663236 Relationships: is a type of plasma membrane protein complex [GO:0098797] Definition: A protein complex that consists of an alphaIIb-beta3 integrin complex bound to talin. Also known as: ITGA2b-ITGB3-TLN1 complex